toll-like receptor 7 signaling pathway [GO:0034154] (biological process) Relationships: is a type of endolysosomal toll-like receptor signaling pathway [GO:0140894] Also known as: TLR7 signaling pathway, toll-like receptor 7 signalling pathway Regulation: regulated by regulation of toll-like receptor 7 signaling pathway [GO:0034155]; negatively regulated by GO:0034156; positively regulated by positive regulation of toll-like receptor 7 signaling pathway [GO:0034157] References: PMID:16551253, PMID:17328678 Sources: GOC:add Definition: The series of molecular signals initiated by a ligand binding to the endolysosomal toll-like receptor 7.